{
  "gene_symbol": "SNRNP35",
  "term_id": "GO:0003729",
  "term_label": "mRNA binding",
  "gene_name": "U11_U12 small nuclear ribonucleoprotein 35 kDa protein",
  "gene": "UniProtKB:Q16560"
}